{
  "term_label": "DNA synthesis involved in UV-damage excision repair",
  "gene_symbol": "POLD3",
  "gene_name": "DNA polymerase delta subunit 3",
  "term_id": "GO:1904161",
  "gene": "UniProtKB:Q15054"
}